{
  "term_id": "GO:0005737",
  "gene": "UniProtKB:Q96D46",
  "gene_symbol": "NMD3",
  "term_label": "cytoplasm",
  "gene_name": "60S ribosomal export protein NMD3"
}